{
  "term_id": "UNKNOWN:0002",
  "gene_name": "Glyoxylate reductase_hydroxypyruvate reductase",
  "gene": "UniProtKB:Q9UBQ7",
  "gene_symbol": "GRHPR",
  "term_label": "Unknown biological process"
}